{
  "gene_name": "Activin receptor type-2A",
  "term_label": "activin receptor complex",
  "gene_symbol": "ACVR2A",
  "term_id": "GO:0048179",
  "gene": "UniProtKB:P27037"
}